{
  "term_id": "GO:0005829",
  "gene_symbol": "BPGM",
  "gene_name": "Bisphosphoglycerate mutase",
  "term_label": "cytosol",
  "gene": "UniProtKB:P07738"
}